{
  "gene_name": "Uncharacterized protein C3orf20",
  "term_label": "Unknown cellular component",
  "gene": "UniProtKB:Q8ND61",
  "gene_symbol": "C3orf20",
  "term_id": "UNKNOWN:0003"
}